{
  "gene": "UniProtKB:Q8IXT1",
  "term_label": "cytoplasm",
  "gene_symbol": "DDIAS",
  "gene_name": "DNA damage-induced apoptosis suppressor protein",
  "term_id": "GO:0005737"
}